{
  "term_label": "maturation of LSU-rRNA",
  "gene": "UniProtKB:O95478",
  "gene_name": "Ribosome biogenesis protein NSA2 homolog",
  "gene_symbol": "NSA2",
  "term_id": "GO:0000470"
}